{
  "term_label": "Unknown biological process",
  "gene_symbol": "PIGC",
  "gene_name": "Phosphatidylinositol N-acetylglucosaminyltransferase subunit C",
  "term_id": "UNKNOWN:0002",
  "gene": "UniProtKB:Q92535"
}